{
  "term_label": "synaptic vesicle",
  "term_id": "GO:0008021",
  "gene_name": "Septin-4",
  "gene": "UniProtKB:O43236",
  "gene_symbol": "SEPTIN4"
}